{
  "gene_symbol": "MMP26",
  "term_label": "extracellular space",
  "term_id": "GO:0005615",
  "gene_name": "Matrix metalloproteinase-26",
  "gene": "UniProtKB:Q9NRE1"
}